{
  "gene": "UniProtKB:P04004",
  "term_label": "cell adhesion mediated by integrin",
  "gene_symbol": "VTN",
  "gene_name": "Vitronectin",
  "term_id": "GO:0033627"
}